{
  "gene": "UniProtKB:Q3LI59",
  "gene_symbol": "KRTAP21-2",
  "term_id": "UNKNOWN:0001",
  "term_label": "Unknown molecular function",
  "gene_name": "Keratin-associated protein 21-2"
}